positive regulation of glucose metabolic process [GO:0010907] (biological process) Relationships: is a type of regulation of glucose metabolic process [GO:0010906]; is_a positive regulation of carbohydrate metabolic process [GO:0045913]; is a type of GO:0062013; positively regulates glucose metabolic process [GO:0006006] Subtypes: positive regulation of gluconeogenesis [GO:0045722], positive regulation of glycogen metabolic process [GO:0070875], GO:1904025 Sources: GOC:BHF, GOC:tb Definition: Any process that increases the rate, frequency or extent of glucose metabolism. Glucose metabolic processes are the chemical reactions and pathways involving glucose, the aldohexose gluco-hexose. Also known as: positive regulation of glucose metabolism